{
  "gene_name": "ATP-dependent RNA helicase TDRD9",
  "term_id": "GO:0003723",
  "term_label": "RNA binding",
  "gene_symbol": "TDRD9",
  "gene": "UniProtKB:Q8NDG6"
}